lipoyl(octanoyl) transferase activity [GO:0033819] (molecular function) Definition: Catalysis of the reaction: L-lysyl-[protein] + octanoyl-[ACP] = H+ + holo-[ACP] + N6-octanoyl-L-lysyl-[protein]. Relationships: is a type of acyltransferase activity, transferring groups other than amino-acyl groups [GO:0016747]; is a type of catalytic activity, acting on a protein [GO:0140096] Also known as: lipoate/octanoate transferase activity, lipoyl (octanoyl)-acyl carrier protein:protein transferase activity, lipoyl (octanoyl)-acyl-carrier-protein-protein N-lipoyltransferase activity, octanoyl-acyl carrier protein-protein N-octanoyltransferase activity, octanoyl-acyl-carrier-protein-protein N-octanoyltransferase activity, octanoyl-acyl-carrier-protein:protein N-octanoyltransferase activity, octanoyl transferase activity (acting on glycine-cleavage complex H protein) Sources: RHEA:17665